{
  "term_label": "Unknown biological process",
  "gene_symbol": "IGHJ1",
  "term_id": "UNKNOWN:0002",
  "gene": "UniProtKB:A0A0C4DH62",
  "gene_name": "Immunoglobulin heavy joining 1"
}